{
  "gene_name": "Exosome complex component RRP45",
  "term_id": "GO:0000177",
  "term_label": "cytoplasmic exosome (RNase complex)",
  "gene": "UniProtKB:Q06265",
  "gene_symbol": "EXOSC9"
}